{
  "term_label": "G-protein beta-subunit binding",
  "gene": "UniProtKB:P61952",
  "term_id": "GO:0031681",
  "gene_symbol": "GNG11",
  "gene_name": "Guanine nucleotide-binding protein G(I)_G(S)_G(O) subunit gamma-11"
}